{
  "gene": "UniProtKB:P50542",
  "term_label": "peroxisome matrix targeting signal-1 binding",
  "term_id": "GO:0005052",
  "gene_symbol": "PEX5",
  "gene_name": "Peroxisomal targeting signal 1 receptor"
}